host cell rough endoplasmic reticulum membrane [GO:0044169] (cellular component) Definition: The lipid bilayer surrounding the host cell rough endoplasmic reticulum. Sources: GOC:jl Also known as: host rough endoplasmic reticulum membrane Relationships: is a type of GO:0044167; is part of GO:0044168